peritoneum development [GO:1904820] (biological process) Also known as: peritonaeum development Relationships: is a type of serous membrane development [GO:1904817] References: PMID:15840053 Sources: GOC:TermGenie, GOC:dph, GO_REF:0000094 Definition: The process whose specific outcome is the progression of a peritoneum over time, from its formation to the mature structure.